{
  "gene": "UniProtKB:P0CB48",
  "gene_symbol": "UBTFL6",
  "term_label": "transcription by RNA polymerase I",
  "term_id": "GO:0006360",
  "gene_name": "Putative upstream-binding factor 1-like protein 6"
}